cellular response to glyoxal [GO:0036471] (biological process) Definition: Any process that results in a change in state or activity of a cell (in terms of movement, secretion, enzyme production, gene expression, etc.) as a result of a glyoxal stimulus. Sources: GOC:PARL, GOC:bf Relationships: is_a cellular response to aldehyde [GO:0110096]